{
  "gene_name": "Polyadenylate-binding protein 5",
  "gene_symbol": "PABPC5",
  "gene": "UniProtKB:Q96DU9",
  "term_label": "cytoplasmic stress granule",
  "term_id": "GO:0010494"
}